{
  "gene_symbol": "PPP2R5B",
  "term_id": "GO:0005829",
  "gene": "UniProtKB:Q15173",
  "gene_name": "Serine_threonine-protein phosphatase 2A 56 kDa regulatory subunit beta isoform",
  "term_label": "cytosol"
}